endocardium formation [GO:0060214] (biological process) Relationships: is a type of anatomical structure formation involved in morphogenesis [GO:0048646]; is part of endocardium morphogenesis [GO:0003160] References: PMID:17722983 Sources: GOC:bf, GOC:dph Definition: Formation of the endocardium of the heart. The endocardium is an anatomical structure comprised of an endothelium and an extracellular matrix that forms the innermost layer of tissue of the heart, and lines the heart chambers.